{
  "gene": "UniProtKB:Q4W4Y0",
  "term_id": "GO:0098989",
  "term_label": "NMDA selective glutamate receptor signaling pathway",
  "gene_name": "Uncharacterized protein C14orf28",
  "gene_symbol": "DORIP1"
}